regulation of neurotrophin TRK receptor signaling pathway [GO:0051386] (biological process) Definition: Any process that modulates the frequency, rate or extent of the neurotrophin TRK receptor signaling pathway. Sources: GOC:ai Also known as: regulation of NGF receptor signaling pathway, regulation of NGF receptor signalling pathway, regulation of nerve growth factor receptor signalling pathway, regulation of nerve growth factor receptor signaling pathway Relationships: is a type of regulation of signal transduction [GO:0009966]; is a type of GO:0090287; regulates neurotrophin TRK receptor signaling pathway [GO:0048011] Subtypes: negative regulation of neurotrophin TRK receptor signaling pathway [GO:0051387], positive regulation of neurotrophin TRK receptor signaling pathway [GO:0051388]